regulation of cell projection organization [GO:0031344] (biological process) Definition: Any process that modulates the frequency, rate or extent of a process involved in the formation, arrangement of constituent parts, or disassembly of cell projections. Sources: GOC:mah Also known as: regulation of cell projection organisation, regulation of cell projection organization and biogenesis Relationships: is a type of regulation of cellular component organization [GO:0051128]; regulates cell projection organization [GO:0030030] Subtypes: negative regulation of cell projection organization [GO:0031345], GO:0031346, regulation of cell projection assembly [GO:0060491], regulation of plasma membrane bounded cell projection organization [GO:0120035], GO:0150011